{
  "term_label": "GTPase activator activity",
  "gene_symbol": "RANGAP1",
  "gene": "UniProtKB:P46060",
  "gene_name": "Ran GTPase-activating protein 1",
  "term_id": "GO:0005096"
}